SUMO ligase activity [GO:0061665] (molecular function) Relationships: is a type of SUMO transferase activity [GO:0019789]; is a type of ubiquitin-like protein ligase activity [GO:0061659] Definition: Catalysis of the transfer of SUMO to a substrate protein via the reaction X-SUMO + S = X + S-SUMO, where X is either an E2 or E3 enzyme, the X-SUMO linkage is a thioester bond, and the S-SUMO linkage is an isopeptide bond between the C-terminal amino acid of SUMO and the epsilon-amino group of lysine residues in the substrate. Subtypes: SUMO-ubiquitin ligase activity [GO:0140082] Sources: GOC:dph Also known as: E3